{
  "gene_symbol": "ALS2",
  "gene_name": "Alsin",
  "term_id": "GO:0031267",
  "term_label": "small GTPase binding",
  "gene": "UniProtKB:Q96Q42"
}